{
  "gene_symbol": "RBBP4",
  "gene_name": "Histone-binding protein RBBP4",
  "gene": "UniProtKB:Q09028",
  "term_label": "chromatin remodeling",
  "term_id": "GO:0006338"
}